{
  "term_label": "RNA polymerase II transcription regulatory region sequence-specific DNA binding",
  "gene_name": "Double homeobox protein 4-like protein 4",
  "gene": "UniProtKB:P0CJ87",
  "gene_symbol": "DUX4L4",
  "term_id": "GO:0000977"
}